{
  "term_id": "UNKNOWN:0002",
  "term_label": "Unknown biological process",
  "gene_symbol": "FAM81A",
  "gene": "UniProtKB:Q8TBF8",
  "gene_name": "Protein FAM81A"
}